{
  "term_id": "GO:0005737",
  "gene": "UniProtKB:Q96TC7",
  "term_label": "cytoplasm",
  "gene_symbol": "RMDN3",
  "gene_name": "Regulator of microtubule dynamics protein 3"
}